nuclear-transcribed mRNA catabolic process, 5'-3' exonucleolytic nonsense-mediated decay [GO:0070479] (biological process) References: PMID:18554525 Note: The reason for obsoletion is that this term was an unnecessary grouping term. Also known as: 5'-3' NMD, 5'-3' nonsense-mediated decay, 5'-3' nonsense-mediated mRNA decay, nuclear-transcribed mRNA breakdown, 5'-3' exonucleolytic nonsense-mediated decay, nuclear-transcribed mRNA catabolism, 5'-3' exonucleolytic nonsense-mediated decay, nuclear-transcribed mRNA degradation, 5'-3' exonucleolytic nonsense-mediated decay Definition: The chemical reactions and pathways resulting in the breakdown of the nuclear-transcribed mRNA transcript body of an mRNA in which an amino-acid codon has changed to a nonsense codon; occurs when the 5' end is not protected by a 5'-cap; degradation proceeds in the 5' to 3' direction. Relationships: is a type of nuclear-transcribed mRNA catabolic process, nonsense-mediated decay [GO:0000184]